{
  "term_label": "ciliary basal body",
  "gene_name": "Intraflagellar transport protein 56",
  "gene_symbol": "IFT56",
  "gene": "UniProtKB:A0AVF1",
  "term_id": "GO:0036064"
}